RNA polymerase I general transcription initiation factor binding [GO:0001179] (molecular function) Relationships: is a type of general transcription initiation factor binding [GO:0140296] Sources: GOC:txnOH Also known as: RNA polymerase I transcription factor binding Definition: Binding to an RNA polymerase I transcription factor, a protein required to initiate or regulate transcription by RNA polymerase I.